{
  "gene_symbol": "ACTL8",
  "gene": "UniProtKB:Q9H568",
  "term_id": "GO:0045202",
  "term_label": "synapse",
  "gene_name": "Actin-like protein 8"
}